{
  "term_label": "Unknown molecular function",
  "gene_symbol": "TCEAL8",
  "gene_name": "Transcription elongation factor A protein-like 8",
  "gene": "UniProtKB:Q8IYN2",
  "term_id": "UNKNOWN:0001"
}